{
  "gene_symbol": "PRORP",
  "term_id": "GO:0001682",
  "gene": "UniProtKB:O15091",
  "term_label": "tRNA 5'-leader removal",
  "gene_name": "Mitochondrial ribonuclease P catalytic subunit"
}